negative regulation of chemokine (C-C motif) ligand 6 production [GO:0035532] (biological process) Also known as: negative regulation of CCL6 production, negative regulation of chemokine (C-C motif) ligand 6 secretion Definition: Any process that stops, prevents, or reduces the frequency, rate, or extent of production of chemokine (C-C motif) ligand 6 (CCL6). Relationships: is a type of negative regulation of chemokine production [GO:0032682]; is a type of GO:0035531; negatively regulates chemokine (C-C motif) ligand 6 production [GO:0035530] Sources: GOC:add, GOC:bf